{
  "term_id": "GO:0005615",
  "gene_symbol": "IFNA16",
  "gene_name": "Interferon alpha-16",
  "term_label": "extracellular space",
  "gene": "UniProtKB:P05015"
}